{
  "gene_name": "Nucleoporin p58_p45",
  "gene": "UniProtKB:Q9BVL2",
  "term_id": "UNKNOWN:0002",
  "gene_symbol": "NUP58",
  "term_label": "Unknown biological process"
}